positive regulation of T cell receptor signaling pathway [GO:0050862] (biological process) Relationships: is a type of GO:0050856; is a type of positive regulation of antigen receptor-mediated signaling pathway [GO:0050857]; positively regulates T cell receptor signaling pathway [GO:0050852] Sources: GOC:ai Also known as: positive regulation of T cell receptor signalling pathway, positive regulation of T lymphocyte receptor signaling pathway, positive regulation of T lymphocyte receptor signalling pathway, positive regulation of T-cell receptor signaling pathway, positive regulation of T-lymphocyte receptor signaling pathway, positive regulation of T-lymphocyte receptor signalling pathway, positive regulation of TCR signaling pathway, up regulation of T cell receptor signaling pathway, up-regulation of T cell receptor signaling pathway, upregulation of T cell receptor signaling pathway, activation of T cell receptor signaling pathway, stimulation of T cell receptor signaling pathway Definition: Any process that activates or increases the frequency, rate or extent of signaling pathways initiated by the cross-linking of an antigen receptor on a T cell.